{
  "gene_name": "Mitogen-activated protein kinase kinase kinase 21",
  "gene": "UniProtKB:Q5TCX8",
  "gene_symbol": "MAP3K21",
  "term_label": "signal transduction",
  "term_id": "GO:0007165"
}